positive regulation of female gonad development [GO:2000196] (biological process) Sources: GOC:obol Definition: Any process that activates or increases the frequency, rate or extent of female gonad development. Also known as: positive regulation of ovarian development, positive regulation of ovary development Relationships: is a type of positive regulation of gonad development [GO:1905941]; is a type of GO:2000194; positively regulates female gonad development [GO:0008585] Subtypes: positive regulation of progesterone secretion [GO:2000872]